conidiogenone biosynthetic process [GO:0140879] (biological process) Relationships: is_a diterpenoid biosynthetic process [GO:0016102]; is a type of ketone biosynthetic process [GO:0042181]; is a type of mycotoxin biosynthetic process [GO:0043386]; is a type of GO:1902653 Also known as: conidiogenone anabolism, conidiogenone biosynthesis, conidiogenone formation, conidiogenone synthesis Definition: The chemical reactions and pathways resulting in the formation of conidiogenone , a diterpene known to induce the conidiation. References: PMID:30343633